{
  "term_label": "protein K63-linked ubiquitination",
  "gene_symbol": "UBE2E3",
  "term_id": "GO:0070534",
  "gene_name": "Ubiquitin-conjugating enzyme E2 E3",
  "gene": "UniProtKB:Q969T4"
}